{
  "term_label": "peptidase activity",
  "gene": "UniProtKB:P83111",
  "gene_name": "Serine beta-lactamase-like protein LACTB, mitochondrial",
  "term_id": "GO:0008233",
  "gene_symbol": "LACTB"
}